negative regulation of T-helper 1 cell cytokine production [GO:2000555] (BP) Relationships: is a type of GO:0002725; is a type of negative regulation of T-helper 1 type immune response [GO:0002826]; is_a regulation of T-helper 1 cell cytokine production [GO:2000554]; negatively regulates T-helper 1 cell cytokine production [GO:0035744] Also known as: negative regulation of Th1 cell cytokine production Sources: GOC:obol Definition: Any process that stops, prevents or reduces the frequency, rate or extent of T-helper 1 cell cytokine production.